{
  "gene_symbol": "PRND",
  "gene_name": "Prion-like protein doppel",
  "term_id": "GO:0009897",
  "term_label": "external side of plasma membrane",
  "gene": "UniProtKB:Q9UKY0"
}